{
  "gene_symbol": "KCNC3",
  "term_label": "potassium ion transmembrane transport",
  "term_id": "GO:0071805",
  "gene_name": "Potassium voltage-gated channel subfamily C member 3",
  "gene": "UniProtKB:Q14003"
}